{
  "gene_name": "NAD-dependent protein deacetylase sirtuin-3, mitochondrial",
  "gene_symbol": "SIRT3",
  "gene": "UniProtKB:Q9NTG7",
  "term_id": "UNKNOWN:0002",
  "term_label": "Unknown biological process"
}